{
  "gene_name": "Coatomer subunit beta'",
  "term_label": "intra-Golgi vesicle-mediated transport",
  "gene": "UniProtKB:P35606",
  "gene_symbol": "COPB2",
  "term_id": "GO:0006891"
}